{
  "term_id": "GO:0005778",
  "gene": "UniProtKB:P40855",
  "gene_name": "Peroxisomal biogenesis factor 19",
  "gene_symbol": "PEX19",
  "term_label": "peroxisomal membrane"
}